regulation of salicylic acid biosynthetic process [GO:0080142] (biological process) Sources: GOC:dhl Relationships: is a type of regulation of biosynthetic process [GO:0009889]; is a type of regulation of salicylic acid metabolic process [GO:0010337]; regulates salicylic acid biosynthetic process [GO:0009697] Definition: Any process that modulates the frequency, rate or extent of the chemical reactions and pathways resulting in the formation of salicylic acid.